{
  "term_id": "GO:0048280",
  "term_label": "vesicle fusion with Golgi apparatus",
  "gene_symbol": "YIPF7",
  "gene": "UniProtKB:Q8N8F6",
  "gene_name": "Protein YIPF7"
}